detection of low humidity stimulus involved in sensory perception [GO:0098515] (BP) Relationships: is a type of detection of humidity stimulus involved in sensory perception [GO:0098512]; is a type of detection of low humidity [GO:0098517]; BFO_0000050 sensory perception of low humidity [GO:0098511] Definition: The series of events in which a low humidity stimulus is detected and converted into a molecular signal as a part of the sensory detection of low humidity. References: PMID:18269908 Sources: GOC:dos